{
  "gene": "UniProtKB:Q8NHP7",
  "gene_symbol": "EXD1",
  "gene_name": "piRNA biogenesis protein EXD1",
  "term_id": "GO:0034587",
  "term_label": "piRNA processing"
}